S-methyl-5-thioribose-1-phosphate isomerase activity [GO:0046523] (MF) Relationships: is a type of intramolecular oxidoreductase activity, interconverting aldoses and ketoses [GO:0016861] Also known as: 5-methylthioribose-1-phosphate isomerase activity, 1-PMTR isomerase activity, 1-phospho-5'-S-methylthioribose isomerase activity, 5-methylthio-5-deoxy-D-ribose-1-phosphate ketol-isomerase activity, MTR-1-P isomerase activity, S-methyl-5-thio-5-deoxy-D-ribose-1-phosphate aldose-ketose-isomerase activity, S-methyl-5-thio-5-deoxy-D-ribose-1-phosphate ketol-isomerase activity, S-methyl-5-thio-D-ribose-1-phosphate aldose-ketose-isomerase activity, S-methyl-5-thio-alpha-D-ribose-1-phosphate aldose-ketose-isomerase activity, methylthioribose 1-phosphate isomerase activity Definition: Catalysis of the reaction: S-methyl-5-thio-alpha-D-ribose 1-phosphate = S-methyl-5-thio-D-ribulose 1-phosphate. Sources: RHEA:19989